{
  "gene": "UniProtKB:O60906",
  "gene_name": "Sphingomyelin phosphodiesterase 2",
  "gene_symbol": "SMPD2",
  "term_id": "GO:0030149",
  "term_label": "sphingolipid catabolic process"
}